H-NS complex [GO:1990121] (cellular component) Definition: A multimer of H-NS proteins that is involved in bacterial nucleoid condensation and negative regulation of global gene expression by directly binding to promoter regions. Recognizes both structural and sequence-specific motifs in double-stranded DNA and has binding preference for bent DNA. References: PMID:12592399 Sources: GOC:bhm Also known as: DNA-binding protein H-NS complex, histone-like protein H-NS complex Relationships: is a type of DNA bending complex [GO:1990104]; is part of GO:0005829; is part of GO:0043590